{
  "gene_symbol": "DDX19A",
  "term_id": "GO:0003724",
  "gene": "UniProtKB:Q9NUU7",
  "term_label": "RNA helicase activity",
  "gene_name": "ATP-dependent RNA helicase DDX19A"
}